{
  "gene_symbol": "DZIP3",
  "gene_name": "E3 ubiquitin-protein ligase DZIP3",
  "gene": "UniProtKB:Q86Y13",
  "term_label": "RNA binding",
  "term_id": "GO:0003723"
}